{
  "term_label": "phosphatidylinositol phosphate binding",
  "gene_symbol": "SNX11",
  "gene": "UniProtKB:Q9Y5W9",
  "term_id": "GO:1901981",
  "gene_name": "Sorting nexin-11"
}